{
  "gene": "UniProtKB:Q9Y3C0",
  "term_id": "UNKNOWN:0001",
  "term_label": "Unknown molecular function",
  "gene_symbol": "WASHC3",
  "gene_name": "WASH complex subunit 3"
}